{
  "gene": "UniProtKB:Q16627",
  "term_label": "positive regulation of cell migration",
  "term_id": "GO:0030335",
  "gene_name": "C-C motif chemokine 14",
  "gene_symbol": "CCL14"
}